{
  "gene_name": "ATP synthase protein 8",
  "gene_symbol": "MT-ATP8",
  "gene": "UniProtKB:P03928",
  "term_label": "proton-transporting ATP synthase activity, rotational mechanism",
  "term_id": "GO:0046933"
}